{
  "gene_name": "Centrosomal protein of 78 kDa",
  "term_label": "Unknown molecular function",
  "gene_symbol": "CEP78",
  "term_id": "UNKNOWN:0001",
  "gene": "UniProtKB:Q5JTW2"
}